{
  "term_label": "regulation of neurogenesis",
  "gene_name": "Achaete-scute homolog 2",
  "gene_symbol": "ASCL2",
  "term_id": "GO:0050767",
  "gene": "UniProtKB:Q99929"
}